{
  "term_label": "cytoplasm",
  "term_id": "GO:0005737",
  "gene": "UniProtKB:Q9NY59",
  "gene_symbol": "SMPD3",
  "gene_name": "Sphingomyelin phosphodiesterase 3"
}